negative regulation of alcohol biosynthetic process [GO:1902931] (biological process) Definition: Any process that stops, prevents or reduces the frequency, rate or extent of alcohol biosynthetic process. References: PMID:23332010 Sources: GOC:TermGenie, GOC:mengo_curators, GO_REF:0000058 Also known as: negative regulation of solventogenesis, down regulation of alcohol anabolism, down regulation of alcohol biosynthesis, down regulation of alcohol biosynthetic process, down regulation of alcohol formation, down regulation of alcohol synthesis, down-regulation of alcohol anabolism, down-regulation of alcohol biosynthesis, down-regulation of alcohol biosynthetic process, down-regulation of alcohol formation, down-regulation of alcohol synthesis, downregulation of alcohol anabolism, downregulation of alcohol biosynthesis, downregulation of alcohol biosynthetic process, downregulation of alcohol formation, downregulation of alcohol synthesis, negative regulation of alcohol anabolism, negative regulation of alcohol biosynthesis, negative regulation of alcohol formation, negative regulation of alcohol synthesis, inhibition of alcohol anabolism, inhibition of alcohol biosynthesis, inhibition of alcohol biosynthetic process, inhibition of alcohol formation, inhibition of alcohol synthesis Relationships: is a type of negative regulation of biosynthetic process [GO:0009890]; is a type of GO:0062014; is a type of regulation of alcohol biosynthetic process [GO:1902930]; negatively regulates alcohol biosynthetic process [GO:0046165] Subtypes: negative regulation of ergosterol biosynthetic process [GO:0010895], GO:0010920, negative regulation of aldosterone biosynthetic process [GO:0032348], negative regulation of cholesterol biosynthetic process [GO:0045541], negative regulation of thiamine biosynthetic process [GO:0070624], negative regulation of abscisic acid biosynthetic process [GO:0090359], negative regulation of inositol biosynthetic process [GO:1900089], negative regulation of kojic acid biosynthetic process [GO:1900395], negative regulation of butyryl-CoA catabolic process to butanol [GO:1900498], negative regulation of asperfuranone biosynthetic process [GO:1900638], GO:1902054, GO:2000065